positive regulation of lamellipodium morphogenesis [GO:2000394] (biological process) Relationships: is_a positive regulation of developmental process [GO:0051094]; is a type of positive regulation of lamellipodium organization [GO:1902745]; is a type of regulation of lamellipodium morphogenesis [GO:2000392]; positively regulates lamellipodium morphogenesis [GO:0072673] Sources: GOC:BHF, GOC:mah Definition: Any process that activates or increases the frequency, rate or extent of lamellipodium morphogenesis. Also known as: positive regulation of lamellipodium organization